{
  "gene": "UniProtKB:P04271",
  "gene_symbol": "S100B",
  "term_label": "RAGE receptor binding",
  "gene_name": "Protein S100-B",
  "term_id": "GO:0050786"
}